{
  "gene_name": "Histone-lysine N-methyltransferase SETD1A",
  "gene": "UniProtKB:O15047",
  "gene_symbol": "SETD1A",
  "term_id": "UNKNOWN:0002",
  "term_label": "Unknown biological process"
}